positive regulation of activin receptor signaling pathway [GO:0032927] (biological process) Definition: Any process that activates or increases the frequency, rate or extent of the activity of any activin receptor signaling pathway. Relationships: is a type of regulation of activin receptor signaling pathway [GO:0032925]; is_a positive regulation of transmembrane receptor protein serine/threonine kinase signaling pathway [GO:0090100]; RO_0002213 activin receptor signaling pathway [GO:0032924] Sources: GOC:BHF, GOC:rl Subtypes: GO:0141092 Also known as: positive regulation of activin receptor signalling pathway, up regulation of activin receptor signaling pathway, up-regulation of activin receptor signaling pathway, upregulation of activin receptor signaling pathway, activation of activin receptor signaling pathway, stimulation of activin receptor signaling pathway, positive regulation of activin signaling pathway, positive regulation of activin signalling pathway